{
  "term_id": "GO:0046513",
  "gene_name": "Sphingomyelin synthase-related protein 1",
  "term_label": "ceramide biosynthetic process",
  "gene_symbol": "SAMD8",
  "gene": "UniProtKB:Q96LT4"
}